platelet dense tubular network [GO:0031094] (cellular component) References: PMID:1322202 Definition: A network of membrane-bounded compartments found in blood platelets, where they regulate platelet activation by sequestering or releasing calcium. The dense tubular network exists as thin elongated membranes in resting platelets, and undergoes a major ultrastructural change, to a rounded vesicular form, upon addition of thrombin. Relationships: is a type of intracellular membrane-bounded organelle [GO:0043231]